calcium-dependent protein serine/threonine phosphatase activity [GO:0004723] (molecular function) Relationships: is a type of GO:0004722 Subtypes: GO:0033192 Regulation: RO_0002211 by calcium-dependent protein serine/threonine phosphatase regulator activity [GO:0008597] Also known as: calcium-dependent protein serine/threonine phosphatase, intrinsic catalyst activity, calcineurin Definition: Catalysis of the reactions: protein serine phosphate + H2O = protein serine + phosphate; and protein threonine phosphate + H2O = protein threonine + phosphate. These reactions require the presence of calcium ions. Sources: GOC:mah